regulation of phosphorus metabolic process [GO:0051174] (biological process) Subtypes: regulation of nucleotide metabolic process [GO:0006140], regulation of phosphorus utilization [GO:0006795], positive regulation of phosphorus metabolic process [GO:0010562], negative regulation of phosphorus metabolic process [GO:0010563], regulation of inositol phosphate biosynthetic process [GO:0010919], regulation of dephosphorylation [GO:0035303], GO:0042325, regulation of acyl-CoA biosynthetic process [GO:0050812], regulation of thiamine diphosphate biosynthetic process [GO:0070616], regulation of coenzyme A biosynthetic process [GO:0080020], regulation of UDP-N-acetylglucosamine biosynthetic process [GO:0106278], regulation of butyryl-CoA catabolic process to butanol [GO:1900497], GO:1900500, regulation of sarcinapterin biosynthetic process [GO:1900971], regulation of tatiopterin biosynthetic process [GO:1900974], regulation of tetrapyrrole biosynthetic process from glycine and succinyl-CoA [GO:1901413], regulation of phospholipid metabolic process [GO:1903725] Definition: Any process that modulates the frequency, rate or extent of the chemical reactions and pathways involving phosphorus or compounds containing phosphorus. Relationships: is a type of GO:0019222; regulates phosphorus metabolic process [GO:0006793] Sources: GOC:ai Also known as: regulation of phosphorus metabolism